{
  "gene_name": "Oxysterols receptor LXR-alpha",
  "term_id": "GO:0010883",
  "gene": "UniProtKB:Q13133",
  "term_label": "regulation of lipid storage",
  "gene_symbol": "NR1H3"
}